{
  "gene_name": "Bcl-2-like protein 13",
  "term_label": "membrane",
  "gene_symbol": "BCL2L13",
  "gene": "UniProtKB:Q9BXK5",
  "term_id": "GO:0016020"
}